parathyroid hormone secretion [GO:0035898] (biological process) Relationships: is a type of endocrine hormone secretion [GO:0060986] References: PMID:12171519, PMID:21164021 Sources: GOC:cjm Regulation: regulated by regulation of parathyroid hormone secretion [GO:2000828]; negatively regulated by negative regulation of parathyroid hormone secretion [GO:2000829]; positively regulated by positive regulation of parathyroid hormone secretion [GO:2000830] Also known as: PTH secretion, parathormone secretion, parathyrin secretion Definition: The regulated release of parathyroid hormone into the circulatory system.